{
  "term_id": "GO:0042127",
  "gene_name": "Transforming growth factor beta-1 proprotein",
  "gene": "UniProtKB:P01137",
  "term_label": "regulation of cell population proliferation",
  "gene_symbol": "TGFB1"
}